positive regulation of hair follicle development [GO:0051798] (biological process) Relationships: is a type of GO:0051094; is a type of positive regulation of multicellular organismal process [GO:0051240]; is a type of regulation of hair follicle development [GO:0051797]; positively regulates hair follicle development [GO:0001942] Definition: Any process that activates or increases the frequency, rate or extent of hair follicle development. Subtypes: GO:0048818 Also known as: up regulation of hair follicle development, up-regulation of hair follicle development, upregulation of hair follicle development, activation of hair follicle development, stimulation of hair follicle development Sources: GOC:ai